{
  "gene_name": "Tumor necrosis factor receptor superfamily member 11B",
  "gene_symbol": "TNFRSF11B",
  "gene": "UniProtKB:O00300",
  "term_id": "UNKNOWN:0003",
  "term_label": "Unknown cellular component"
}